{
  "term_id": "GO:0005634",
  "gene_name": "Serine_threonine-protein phosphatase PP1-gamma catalytic subunit",
  "gene": "UniProtKB:P36873",
  "gene_symbol": "PPP1CC",
  "term_label": "nucleus"
}